{
  "gene_name": "Dynactin subunit 1",
  "gene_symbol": "DCTN1",
  "gene": "UniProtKB:Q14203",
  "term_id": "GO:0007097",
  "term_label": "nuclear migration"
}